{
  "gene": "UniProtKB:Q9NP70",
  "term_id": "GO:0007155",
  "term_label": "cell adhesion",
  "gene_name": "Ameloblastin",
  "gene_symbol": "AMBN"
}